{
  "term_id": "GO:0055088",
  "gene_name": "TLC domain-containing protein 4",
  "gene_symbol": "TLCD4",
  "gene": "UniProtKB:Q96MV1",
  "term_label": "lipid homeostasis"
}